cell fate commitment involved in formation of primary germ layer [GO:0060795] (biological process) Subtypes: mesodermal cell fate commitment [GO:0001710], endodermal cell fate commitment [GO:0001711], ectodermal cell fate commitment [GO:0001712] Definition: The commitment of cells to specific cell fates of the endoderm, ectoderm, or mesoderm as a part of gastrulation. Sources: GOC:dph, GOC:sdb_2009, GOC:tb Relationships: is a type of cell fate commitment [GO:0045165]; is part of GO:0001704